{
  "gene": "UniProtKB:Q96SI9",
  "term_label": "Unknown biological process",
  "term_id": "UNKNOWN:0002",
  "gene_symbol": "STRBP",
  "gene_name": "Spermatid perinuclear RNA-binding protein"
}